{
  "term_id": "UNKNOWN:0002",
  "term_label": "Unknown biological process",
  "gene": "UniProtKB:P0C7N8",
  "gene_symbol": "OR9G9",
  "gene_name": "Olfactory receptor 9G9"
}